regulation of gibberellic acid mediated signaling pathway [GO:0009937] (BP) Definition: Any process that modulates the frequency, rate or extent of gibberellic acid mediated signaling. Also known as: regulation of gibberellic acid mediated signalling Relationships: is_a regulation of signal transduction [GO:0009966]; regulates gibberellic acid mediated signaling pathway [GO:0009740] Subtypes: GO:0009938, positive regulation of gibberellic acid mediated signaling pathway [GO:0009939] Sources: GOC:go_curators